{
  "gene_symbol": "TRAF3IP2",
  "gene": "UniProtKB:O43734",
  "gene_name": "E3 ubiquitin ligase TRAF3IP2",
  "term_label": "humoral immune response",
  "term_id": "GO:0006959"
}